{
  "term_label": "cellular response to nutrient levels",
  "term_id": "GO:0031669",
  "gene": "UniProtKB:Q969E3",
  "gene_name": "Urocortin-3",
  "gene_symbol": "UCN3"
}